{
  "term_label": "Unknown molecular function",
  "gene_name": "Surfeit locus protein 4",
  "term_id": "UNKNOWN:0001",
  "gene": "UniProtKB:O15260",
  "gene_symbol": "SURF4"
}